{
  "gene": "UniProtKB:Q9UPN7",
  "gene_symbol": "PPP6R1",
  "term_label": "regulation of signal transduction",
  "term_id": "GO:0009966",
  "gene_name": "Serine_threonine-protein phosphatase 6 regulatory subunit 1"
}